{
  "term_label": "nucleus",
  "gene": "UniProtKB:Q9Y4A5",
  "term_id": "GO:0005634",
  "gene_symbol": "TRRAP",
  "gene_name": "Transformation_transcription domain-associated protein"
}